{
  "term_id": "GO:0005634",
  "gene_name": "Protein argonaute-1",
  "gene_symbol": "AGO1",
  "gene": "UniProtKB:Q9UL18",
  "term_label": "nucleus"
}